{
  "term_id": "GO:0042626",
  "term_label": "ATPase-coupled transmembrane transporter activity",
  "gene": "UniProtKB:Q9NUT2",
  "gene_name": "Mitochondrial potassium channel ATP-binding subunit",
  "gene_symbol": "ABCB8"
}